post-embryonic forelimb morphogenesis [GO:0035128] (biological process) Sources: GOC:bf Relationships: is a type of post-embryonic limb morphogenesis [GO:0035127]; is a type of GO:0035136 Definition: The process, occurring after embryonic development, by which the anatomical structures of the forelimb are generated and organized. The forelimbs are the front limbs of an organism.